{
  "gene_name": "Persulfide dioxygenase ETHE1, mitochondrial",
  "term_label": "hydrogen sulfide metabolic process",
  "gene": "UniProtKB:O95571",
  "term_id": "GO:0070813",
  "gene_symbol": "ETHE1"
}